{
  "gene_symbol": "RNF185",
  "gene_name": "E3 ubiquitin-protein ligase RNF185",
  "gene": "UniProtKB:Q96GF1",
  "term_id": "GO:0036503",
  "term_label": "ERAD pathway"
}